{
  "gene": "UniProtKB:P01024",
  "gene_name": "Complement C3",
  "term_label": "extracellular space",
  "term_id": "GO:0005615",
  "gene_symbol": "C3"
}